{
  "term_label": "eukaryotic 43S preinitiation complex",
  "gene": "UniProtKB:O15372",
  "term_id": "GO:0016282",
  "gene_symbol": "EIF3H",
  "gene_name": "Eukaryotic translation initiation factor 3 subunit H"
}